{
  "gene_symbol": "VPS13B",
  "term_id": "UNKNOWN:0002",
  "gene": "UniProtKB:Q7Z7G8",
  "term_label": "Unknown biological process",
  "gene_name": "Intermembrane lipid transfer protein VPS13B"
}